MHC protein binding [GO:0042287] (molecular function) Definition: Binding to a major histocompatibility complex molecule; a set of molecules displayed on cell surfaces that are responsible for lymphocyte recognition and antigen presentation. Also known as: major histocompatibility complex binding, major histocompatibility complex ligand Subtypes: MHC class Ib protein binding [GO:0023029], MHC class I protein binding [GO:0042288], GO:0042289 Note: Note that this term does not include binding to the antigen peptide bound to the MHC protein, for this also annotate to 'peptide antigen binding ; GO:0042605' or one of its children. Sources: GOC:jl Relationships: is a type of GO:0005102